{
  "gene_name": "Origin recognition complex subunit 2",
  "term_label": "nuclear origin of replication recognition complex",
  "gene_symbol": "ORC2",
  "term_id": "GO:0005664",
  "gene": "UniProtKB:Q13416"
}